{
  "gene": "UniProtKB:O00587",
  "term_label": "O-fucosylpeptide 3-beta-N-acetylglucosaminyltransferase activity",
  "term_id": "GO:0033829",
  "gene_name": "Beta-1,3-N-acetylglucosaminyltransferase manic fringe",
  "gene_symbol": "MFNG"
}